{
  "gene": "UniProtKB:P05014",
  "term_id": "GO:0002312",
  "term_label": "B cell activation involved in immune response",
  "gene_symbol": "IFNA4",
  "gene_name": "Interferon alpha-4"
}